{
  "term_id": "GO:0005791",
  "gene": "UniProtKB:O95237",
  "gene_symbol": "LRAT",
  "term_label": "rough endoplasmic reticulum",
  "gene_name": "Lecithin retinol acyltransferase"
}